carotenoid biosynthetic process [GO:0016117] (biological process) Also known as: carotenoid anabolism, carotenoid biosynthesis, carotenoid formation, carotenoid synthesis Definition: The chemical reactions and pathways resulting in the formation of carotenoids, tetraterpenoid compounds in which two units of 4 isoprenoid residues joined head-to-tail are themselves joined tail-to-tail. Relationships: is a type of tetraterpenoid biosynthetic process [GO:0016109]; is a type of carotenoid metabolic process [GO:0016116]; is a type of pigment biosynthetic process [GO:0046148] Regulation: negatively regulated by negative regulation of carotenoid biosynthetic process [GO:1904142]; positively regulated by GO:1904143 Subtypes: xanthophyll biosynthetic process [GO:0016123], beta-carotene biosynthetic process [GO:1901812], GO:1901818, alpha-zeacarotene biosynthetic process [GO:1901821], alpha-carotene biosynthetic process [GO:1901824], zeaxanthin bis(beta-D-glucoside) biosynthetic process [GO:1901830] Sources: GOC:go_curators